{
  "term_id": "UNKNOWN:0002",
  "gene_name": "Heat shock protein beta-9",
  "term_label": "Unknown biological process",
  "gene": "UniProtKB:Q9BQS6",
  "gene_symbol": "HSPB9"
}